tyrosyl-RNA phosphodiesterase activity [GO:0036317] (molecular function) References: PMID:21408223, PMID:22908287 Sources: GOC:bf, GOC:sp Also known as: VPg unlinkase activity, Y-pUpN PDE activity, unlinkase activity, uridylylpolynucleotide-(5' P->O)- tyrosine phosphodiesterase activity Relationships: is a type of GO:0008081; is a type of catalytic activity, acting on RNA [GO:0140098] Definition: Catalysis of the hydrolysis of a 5' tyrosyl-RNA phosphodiester bond between a protein and RNA. In picornaviruses, this covalent bond connects VPg, a viral-encoded protein essential for RNA replication, to the 5' end of all nascent picornavirus genomes; it is cleaved from viral RNA prior to its engaging in protein synthesis.